negative regulation of stress fiber assembly [GO:0051497] (BP) Definition: Any process that stops, prevents, or reduces the frequency, rate or extent of the assembly a stress fiber, a bundle of microfilaments and other proteins found in fibroblasts. Sources: GOC:ai Also known as: down-regulation of stress fiber formation, inhibition of stress fiber formation, down regulation of stress fiber formation, downregulation of stress fiber formation, negative regulation of stress fibre biosynthesis, negative regulation of stress fibre formation Relationships: is a type of negative regulation of actin filament bundle assembly [GO:0032232]; is a type of regulation of stress fiber assembly [GO:0051492]; negatively regulates GO:0043149